microtubule severing [GO:0051013] (biological process) References: PMID:27037673 Sources: GOC:ai Relationships: is a type of microtubule cytoskeleton organization [GO:0000226] Also known as: microtubule severing activity Definition: The process in which a microtubule is broken down into smaller segments. Severing enzymes remove dimers from the middle of the filament to create new ends, unlike depolymerizing kinesins that use ATP to uncap microtubules at their ends.